{
  "gene": "UniProtKB:Q8NEG2",
  "term_id": "UNKNOWN:0003",
  "gene_symbol": "C7orf57",
  "gene_name": "Uncharacterized protein C7orf57",
  "term_label": "Unknown cellular component"
}